{
  "term_id": "UNKNOWN:0003",
  "gene_name": "Uncharacterized protein C9orf85",
  "gene": "UniProtKB:Q96MD7",
  "term_label": "Unknown cellular component",
  "gene_symbol": "C9orf85"
}